epoxide hydrolase activity [GO:0004301] (molecular function) Also known as: arene-oxide hydratase activity, aryl epoxide hydrase activity, epoxide hydrase activity, epoxide hydratase activity, soluble epoxide hydrolase activity, cytosolic epoxide hydrolase activity, sEH, trans-stilbene oxide hydrolase activity Relationships: is a type of ether hydrolase activity [GO:0016803] Definition: Catalysis of the reaction: an epoxide + H2O = an ethanediol. Subtypes: juvenile hormone epoxide hydrolase activity [GO:0008096], GO:0018744, phenanthrene-epoxide hydrolase activity [GO:0019118], GO:0033961, GO:0047977 Sources: EC:3.3.2.10